{
  "gene_symbol": "PPL",
  "term_id": "GO:0042060",
  "term_label": "wound healing",
  "gene_name": "Periplakin",
  "gene": "UniProtKB:O60437"
}